{
  "term_id": "GO:0006357",
  "gene_symbol": "ZBED6",
  "gene_name": "Zinc finger BED domain-containing protein 6",
  "term_label": "regulation of transcription by RNA polymerase II",
  "gene": "UniProtKB:P86452"
}